{
  "term_label": "membrane",
  "gene": "UniProtKB:Q9BWQ8",
  "gene_symbol": "FAIM2",
  "term_id": "GO:0016020",
  "gene_name": "Protein lifeguard 2"
}